{
  "term_label": "respiratory chain complex III",
  "gene_symbol": "CYC1",
  "term_id": "GO:0045275",
  "gene": "UniProtKB:P08574",
  "gene_name": "Cytochrome c1, heme protein, mitochondrial"
}